protein localization to centriolar satellite [GO:0120329] (biological process) Also known as: protein localisation to centriolar satellite Definition: A process in which a protein is transported to, or maintained in, a location within a centriolar satellite. Relationships: is a type of protein localization to centrosome [GO:0071539] References: PMID:34782749